hydroxylamine reductase (NADH) activity [GO:0050460] (molecular function) Definition: Catalysis of the reaction: NH4+ + NAD+ + H2O = hydroxylamine + NADH + 2 H+. Sources: RHEA:20581 Also known as: N-hydroxy amine reductase activity, NADH-hydroxylamine reductase activity, NADH2:hydroxylamine oxidoreductase activity, NADH:hydroxylamine oxidoreductase activity, ammonium dehydrogenase activity, ammonium:NAD+ oxidoreductase activity, hydroxylamine reductase (NADH2) Relationships: is a type of oxidoreductase activity, acting on other nitrogenous compounds as donors, with NAD or NADP as acceptor [GO:0046857]